{
  "term_label": "U12-type spliceosomal complex",
  "gene": "UniProtKB:Q9UK45",
  "gene_name": "U6 snRNA-associated Sm-like protein LSm7",
  "term_id": "GO:0005689",
  "gene_symbol": "LSM7"
}